pore formation during contractile vacuole discharge [GO:0140028] (biological process) Definition: The formation of a transient pore in the plasma membrane and the attached contractile vacuolar membrane, to release water from the cell. This process does not involve fusion of the two membranes. Relationships: is a type of exocytic process [GO:0140029]; is part of contractile vacuole discharge [GO:0070177] References: PMID:22323285 Sources: Wikipedia:Exocytosis